{
  "gene_name": "Iroquois-class homeodomain protein IRX-2",
  "term_id": "GO:0030182",
  "gene_symbol": "IRX2",
  "term_label": "neuron differentiation",
  "gene": "UniProtKB:Q9BZI1"
}